acetylcholine secretion [GO:0061526] (biological process) Relationships: is_a acetylcholine transport [GO:0015870]; is a type of signal release [GO:0023061] Sources: GOC:dph Subtypes: acetylcholine secretion, neurotransmission [GO:0014055] Definition: The regulated release of acetylcholine by a cell.